{
  "term_id": "GO:0006226",
  "gene_symbol": "DUT",
  "term_label": "dUMP biosynthetic process",
  "gene": "UniProtKB:P33316",
  "gene_name": "Deoxyuridine 5'-triphosphate nucleotidohydrolase, mitochondrial"
}